synaptic vesicle to endosome fusion [GO:0016189] (biological process) Note: This covers fusion of synaptic vesicles trafficked to the synapse as well as fusion of endocytosed vesicles as part of recycling. It is there for not part of the synaptic vesicle cycle. Definition: Fusion of a synaptic vesicle with an endosome. Relationships: is a type of endosome organization [GO:0007032]; is a type of GO:0048284; is part of synaptic vesicle endosomal processing [GO:0099532] References: PMID:10099709 Sources: GOC:curators Subtypes: endocytosed synaptic vesicle to endosome fusion [GO:0099593]